{
  "gene_symbol": "ITPKB",
  "gene_name": "Inositol-trisphosphate 3-kinase B",
  "gene": "UniProtKB:P27987",
  "term_id": "GO:0005634",
  "term_label": "nucleus"
}